camphene synthase activity [GO:0102703] (MF) Definition: Catalysis of the reaction: geranyl diphosphate = (-)-camphene + diphosphoric acid. Sources: EC:4.2.3.117, GOC:pz Relationships: is a type of carbon-oxygen lyase activity, acting on phosphates [GO:0016838]